phosphopyruvate hydratase complex [GO:0000015] (cellular component) Also known as: enolase complex Relationships: is a type of catalytic complex [GO:1902494]; is part of cytosol [GO:0005829] Definition: A multimeric enzyme complex, usually a dimer or an octamer, that catalyzes the conversion of 2-phospho-D-glycerate to phosphoenolpyruvate and water. Sources: GOC:jl, ISBN:0198506732